{
  "term_id": "GO:0007399",
  "gene_name": "Protein unc-119 homolog A",
  "gene": "UniProtKB:Q13432",
  "gene_symbol": "UNC119",
  "term_label": "nervous system development"
}